epithelial structure maintenance [GO:0010669] (biological process) Sources: GOC:dph, GOC:tb Definition: A tissue homeostatic process required for the maintenance of epithelial structure. Relationships: is a type of GO:0001894 Subtypes: maintenance of gastrointestinal epithelium [GO:0030277], GO:0035160